{
  "gene_name": "Importin-8",
  "term_label": "cytosol",
  "term_id": "GO:0005829",
  "gene_symbol": "IPO8",
  "gene": "UniProtKB:O15397"
}